plant endodermal cell differentiation [GO:0160058] (biological process) References: PMID:21735349 Definition: The process in which a relatively unspecialized cell acquires specialized features of a plant endodermal cell. Relationships: is a type of cell differentiation [GO:0030154]